{
  "term_label": "cytoplasm",
  "gene_symbol": "DNA2",
  "term_id": "GO:0005737",
  "gene": "UniProtKB:P51530",
  "gene_name": "DNA replication ATP-dependent helicase_nuclease DNA2"
}